{
  "gene_name": "Ras-related protein Rab-42",
  "term_id": "GO:0007264",
  "gene_symbol": "RAB42",
  "term_label": "small GTPase-mediated signal transduction",
  "gene": "UniProtKB:Q8N4Z0"
}